{
  "gene_name": "Cysteine-rich protein 3",
  "term_id": "UNKNOWN:0001",
  "gene": "UniProtKB:Q6Q6R5",
  "gene_symbol": "CRIP3",
  "term_label": "Unknown molecular function"
}